{
  "term_label": "Golgi membrane",
  "gene_name": "Bombesin receptor-activated protein C6orf89",
  "term_id": "GO:0000139",
  "gene": "UniProtKB:Q6UWU4",
  "gene_symbol": "C6orf89"
}